{
  "gene_symbol": "TASOR2",
  "term_id": "UNKNOWN:0002",
  "gene": "UniProtKB:Q5VWN6",
  "gene_name": "Protein TASOR 2",
  "term_label": "Unknown biological process"
}